regulation of platelet-derived growth factor receptor-beta signaling pathway [GO:2000586] (biological process) Sources: GOC:obol Relationships: is a type of GO:0010640; regulates platelet-derived growth factor receptor-beta signaling pathway [GO:0035791] Also known as: regulation of PDGF receptor-beta signaling pathway, regulation of PDGFR-beta signaling pathway, regulation of betaPDGF receptor signaling pathway, regulation of platelet-derived growth factor receptor-beta signalling pathway Definition: Any process that modulates the frequency, rate or extent of platelet-derived growth factor receptor-beta signaling pathway. Subtypes: GO:2000587, positive regulation of platelet-derived growth factor receptor-beta signaling pathway [GO:2000588]